positive regulation of vascular permeability [GO:0043117] (biological process) Also known as: up regulation of vascular permeability, up-regulation of vascular permeability, upregulation of vascular permeability, activation of vascular permeability, stimulation of vascular permeability Sources: GOC:jl Definition: Any process that increases the extent to which blood vessels can be pervaded by fluid. Subtypes: positive regulation of blood-brain barrier permeability [GO:1905605] Relationships: is a type of regulation of vascular permeability [GO:0043114]